{
  "gene": "UniProtKB:P16885",
  "gene_symbol": "PLCG2",
  "gene_name": "1-phosphatidylinositol 4,5-bisphosphate phosphodiesterase gamma-2",
  "term_label": "release of sequestered calcium ion into cytosol",
  "term_id": "GO:0051209"
}